{
  "gene": "UniProtKB:A8MTY0",
  "term_id": "GO:0000981",
  "gene_symbol": "ZNF724",
  "gene_name": "Zinc finger protein 724",
  "term_label": "DNA-binding transcription factor activity, RNA polymerase II-specific"
}